{
  "gene": "UniProtKB:Q96P44",
  "gene_name": "Collagen alpha-1(XXI) chain",
  "term_id": "UNKNOWN:0001",
  "term_label": "Unknown molecular function",
  "gene_symbol": "COL21A1"
}